negative regulation of sperm capacitation [GO:1902491] (biological process) References: PMID:22539676 Sources: GOC:TermGenie, GOC:hjd Relationships: is a type of negative regulation of multicellular organismal process [GO:0051241]; is a type of regulation of sperm capacitation [GO:1902490]; is a type of negative regulation of cell maturation [GO:1903430]; is a type of negative regulation of reproductive process [GO:2000242]; negatively regulates sperm capacitation [GO:0048240] Definition: Any process that stops, prevents or reduces the frequency, rate or extent of sperm capacitation. Also known as: down regulation of sperm capacitation, down-regulation of sperm capacitation, downregulation of sperm capacitation, inhibition of sperm capacitation, down regulation of sperm activation, down-regulation of sperm activation, downregulation of sperm activation, inhibition of sperm activation, negative regulation of sperm activation